{
  "gene": "UniProtKB:P15151",
  "term_label": "virus receptor activity",
  "gene_symbol": "PVR",
  "term_id": "GO:0001618",
  "gene_name": "Poliovirus receptor"
}